{
  "term_label": "Unknown molecular function",
  "gene": "UniProtKB:P53618",
  "term_id": "UNKNOWN:0001",
  "gene_name": "Coatomer subunit beta",
  "gene_symbol": "COPB1"
}